{
  "term_label": "lysosome",
  "gene": "UniProtKB:Q96AX1",
  "term_id": "GO:0005764",
  "gene_name": "Vacuolar protein sorting-associated protein 33A",
  "gene_symbol": "VPS33A"
}